{
  "term_label": "synaptic vesicle membrane",
  "term_id": "GO:0030672",
  "gene_name": "Vesicular glutamate transporter 2",
  "gene_symbol": "SLC17A6",
  "gene": "UniProtKB:Q9P2U8"
}